{
  "gene": "UniProtKB:O75943",
  "gene_symbol": "RAD17",
  "term_id": "GO:0031573",
  "term_label": "mitotic intra-S DNA damage checkpoint signaling",
  "gene_name": "Cell cycle checkpoint protein RAD17"
}